positive regulation of cellobiose catabolic process [GO:1900284] (biological process) Relationships: is a type of positive regulation of catabolic process [GO:0009896]; is a type of positive regulation of carbohydrate metabolic process [GO:0045913]; is a type of regulation of cellobiose catabolic process [GO:1900282]; RO_0002213 cellobiose catabolic process [GO:2000892] Definition: Any process that activates or increases the frequency, rate or extent of cellobiose catabolic process. Sources: GOC:TermGenie, GOC:mengo_curators Also known as: positive regulation of cellobiose catabolism, up regulation of cellobiose catabolic process, up regulation of cellobiose catabolism, up-regulation of cellobiose catabolic process, up-regulation of cellobiose catabolism, upregulation of cellobiose catabolic process, upregulation of cellobiose catabolism, activation of cellobiose catabolic process, activation of cellobiose catabolism